{
  "gene_name": "NADH dehydrogenase (ubiquinone) complex I, assembly factor 6",
  "term_id": "GO:0005739",
  "gene_symbol": "NDUFAF6",
  "term_label": "mitochondrion",
  "gene": "UniProtKB:Q330K2"
}